{
  "gene": "UniProtKB:Q9Y5A7",
  "gene_name": "NEDD8 ultimate buster 1",
  "term_id": "GO:2000058",
  "term_label": "regulation of ubiquitin-dependent protein catabolic process",
  "gene_symbol": "NUB1"
}